{
  "term_id": "UNKNOWN:0003",
  "term_label": "Unknown cellular component",
  "gene_name": "Putative uncharacterized protein PP632",
  "gene_symbol": "PP632",
  "gene": "UniProtKB:Q6XCG6"
}